{
  "gene_symbol": "APOO",
  "gene_name": "MICOS complex subunit MIC26",
  "gene": "UniProtKB:Q9BUR5",
  "term_label": "Unknown molecular function",
  "term_id": "UNKNOWN:0001"
}